regulation of plant organ formation [GO:1905428] (biological process) Sources: GOC:TermGenie, GOC:tb, GO_REF:0000058 Subtypes: regulation of timing of plant organ formation [GO:0090709], regulation of leaf formation [GO:2000025], regulation of secondary shoot formation [GO:2000032] Definition: Any process that modulates the frequency, rate or extent of plant organ formation. Relationships: is a type of regulation of anatomical structure morphogenesis [GO:0022603]; regulates plant organ formation [GO:1905393]